{
  "gene_name": "Receptor-interacting serine_threonine-protein kinase 2",
  "term_id": "GO:0045087",
  "gene_symbol": "RIPK2",
  "term_label": "innate immune response",
  "gene": "UniProtKB:O43353"
}